negative regulation of response to cycloalkane [GO:1901432] (biological process) Also known as: down regulation of response to cycloalkane, down-regulation of response to cycloalkane, downregulation of response to cycloalkane, inhibition of response to cycloalkane Definition: Any process that stops, prevents or reduces the frequency, rate or extent of response to cycloalkane. Sources: GOC:TermGenie, GOC:mengo_curators Relationships: is a type of negative regulation of response to stimulus [GO:0048585]; is a type of regulation of response to cycloalkane [GO:1901431]; negatively regulates response to cycloalkane [GO:0014071]